{
  "term_id": "UNKNOWN:0001",
  "gene_symbol": "MED10",
  "gene_name": "Mediator of RNA polymerase II transcription subunit 10",
  "term_label": "Unknown molecular function",
  "gene": "UniProtKB:Q9BTT4"
}